{
  "gene": "UniProtKB:Q13617",
  "gene_symbol": "CUL2",
  "term_id": "GO:0005737",
  "gene_name": "Cullin-2",
  "term_label": "cytoplasm"
}